{
  "gene_name": "Occludin",
  "gene_symbol": "OCLN",
  "gene": "UniProtKB:Q16625",
  "term_label": "bicellular tight junction assembly",
  "term_id": "GO:0070830"
}